{
  "gene": "UniProtKB:Q9H300",
  "term_label": "serine-type endopeptidase activity",
  "gene_name": "Presenilin-associated rhomboid-like protein, mitochondrial",
  "term_id": "GO:0004252",
  "gene_symbol": "PARL"
}